{
  "gene_name": "NPC1-like intracellular cholesterol transporter 1",
  "term_label": "intestinal cholesterol absorption",
  "gene": "UniProtKB:Q9UHC9",
  "term_id": "GO:0030299",
  "gene_symbol": "NPC1L1"
}